interphase SIN signaling complex [GO:0160066] (cellular component) Definition: A SIN signaling complex associated with the old mitotic spindle pole body during interphase and early M-phase and characterised by the presence active ubiquitin ligase (Dma1 in fission yeast) and GTPase activator (Spg1 in fission yeast) to inactivate SIN signaling. References: PMID:21131906 Also known as: interphase SIN signalling complex Relationships: is a type of SIN/MEN signaling complex [GO:0160065]